{
  "term_id": "GO:0030956",
  "term_label": "glutamyl-tRNA(Gln) amidotransferase complex",
  "gene": "UniProtKB:O43716",
  "gene_symbol": "GATC",
  "gene_name": "Glutamyl-tRNA(Gln) amidotransferase subunit C, mitochondrial"
}